{
  "gene_name": "FH1_FH2 domain-containing protein 3",
  "gene": "UniProtKB:Q2V2M9",
  "gene_symbol": "FHOD3",
  "term_label": "cardiac myofibril assembly",
  "term_id": "GO:0055003"
}